{
  "term_id": "GO:0051014",
  "term_label": "actin filament severing",
  "gene_name": "Cofilin-1",
  "gene": "UniProtKB:P23528",
  "gene_symbol": "CFL1"
}